{
  "term_label": "calcium ion binding",
  "gene_symbol": "CALML4",
  "gene": "UniProtKB:Q96GE6",
  "term_id": "GO:0005509",
  "gene_name": "Calmodulin-like protein 4"
}